{
  "gene_name": "Cell cycle and apoptosis regulator protein 2",
  "term_label": "Unknown biological process",
  "gene": "UniProtKB:Q8N163",
  "term_id": "UNKNOWN:0002",
  "gene_symbol": "CCAR2"
}